{
  "gene_name": "YY1-associated protein 1",
  "gene": "UniProtKB:Q9H869",
  "term_id": "UNKNOWN:0001",
  "term_label": "Unknown molecular function",
  "gene_symbol": "YY1AP1"
}